phenylacetaldehyde synthase activity [GO:1990055] (molecular function) References: PMID:16766535, PMID:23204519 Sources: RHEA:55532 Relationships: is a type of GO:0016831 Also known as: aromatic aldehyde synthase Definition: Catalyzes the reaction: L-phenylalanine + O2 + H2O + H+ = 2-phenylacetaldehyde + H2O2 + NH4+ + CO2.